{
  "gene_symbol": "REPS1",
  "gene_name": "RalBP1-associated Eps domain-containing protein 1",
  "gene": "UniProtKB:Q96D71",
  "term_label": "endosomal transport",
  "term_id": "GO:0016197"
}